{
  "gene_name": "Slit homolog 3 protein",
  "term_label": "heparin binding",
  "term_id": "GO:0008201",
  "gene": "UniProtKB:O75094",
  "gene_symbol": "SLIT3"
}